{
  "gene_symbol": "ELOVL5",
  "term_id": "GO:0009922",
  "gene": "UniProtKB:Q9NYP7",
  "term_label": "fatty acid elongase activity",
  "gene_name": "Elongation of very long chain fatty acids protein 5"
}